FAT10 activating enzyme activity [GO:0019780] (molecular function) Sources: GOC:mah Relationships: is a type of ubiquitin-like modifier activating enzyme activity [GO:0008641] Definition: Catalysis of the activation of the small ubiquitin-related modifier FAT10, through the formation of an ATP-dependent high-energy thiolester bond.